{
  "term_id": "GO:0048012",
  "gene_symbol": "HGF",
  "gene": "UniProtKB:P14210",
  "term_label": "hepatocyte growth factor receptor signaling pathway",
  "gene_name": "Hepatocyte growth factor"
}